{
  "term_label": "cytidine deaminase activity",
  "gene_symbol": "APOBEC3D",
  "gene": "UniProtKB:Q96AK3",
  "gene_name": "DNA dC-dU-editing enzyme APOBEC-3D",
  "term_id": "GO:0004126"
}